{
  "gene_name": "TNF receptor-associated factor 6",
  "term_label": "lipopolysaccharide-mediated signaling pathway",
  "gene": "UniProtKB:Q9Y4K3",
  "gene_symbol": "TRAF6",
  "term_id": "GO:0031663"
}